regulation of hemoglobin biosynthetic process [GO:0046984] (biological process) Subtypes: positive regulation of hemoglobin biosynthetic process [GO:0046985], GO:0046986 Relationships: is a type of GO:0010556; is a type of regulation of protein metabolic process [GO:0051246]; regulates GO:0042541 Sources: GOC:ai Also known as: regulation of haemoglobin biosynthesis, regulation of haemoglobin biosynthetic process, regulation of hemoglobin anabolism, regulation of hemoglobin biosynthesis, regulation of hemoglobin formation, regulation of hemoglobin synthesis Definition: Any process that modulates the frequency, rate or extent of the chemical reactions and pathways resulting in the formation of hemoglobin, an oxygen carrying, conjugated protein containing four heme groups and globin.